{
  "term_label": "Unknown cellular component",
  "term_id": "UNKNOWN:0003",
  "gene": "UniProtKB:Q9Y694",
  "gene_symbol": "SLC22A7",
  "gene_name": "Solute carrier family 22 member 7"
}